CCR4-NOT complex [GO:0030014] (cellular component) References: PMID:11113136, PMID:11239395, PMID:22785621, PMID:30601114 Sources: GOC:sart Definition: The Ccr4-Not complex is an eukaryotically conserved deadenylase that can initiate cytoplasmic mRNA decay, and reduce translation by releasing poly(A)-binding protein (Pab1/PABPC1). Ccr4-Not contains seven core subunits, including two poly(A)-specific exonucleases, Ccr4/CNOT6/CNOT6L and Caf1/Pop2/CNOT7/CNOT8. Relationships: is a type of intracellular protein-containing complex [GO:0140535]